{
  "gene_name": "Importin subunit alpha-5",
  "gene_symbol": "KPNA1",
  "term_id": "GO:0006607",
  "gene": "UniProtKB:P52294",
  "term_label": "NLS-bearing protein import into nucleus"
}